{
  "gene_symbol": "DHX58",
  "gene_name": "ATP-dependent RNA helicase DHX58",
  "term_label": "cytoplasmic pattern recognition receptor signaling pathway",
  "term_id": "GO:0002753",
  "gene": "UniProtKB:Q96C10"
}